{
  "gene_name": "Serpin H1",
  "term_label": "serine-type endopeptidase inhibitor activity",
  "term_id": "GO:0004867",
  "gene": "UniProtKB:P50454",
  "gene_symbol": "SERPINH1"
}